regulation of invasive growth in response to glucose limitation [GO:2000217] (biological process) Relationships: is a type of GO:0070784; RO_0002211 invasive growth in response to glucose limitation [GO:0001403] Sources: GOC:mah Subtypes: GO:2000218, positive regulation of invasive growth in response to glucose limitation [GO:2000219] Definition: Any process that modulates the frequency, rate or extent of invasive growth in response to glucose limitation. Also known as: regulation of colony morphology